chondrocyte intercalation involved in growth plate cartilage morphogenesis [GO:0003428] (biological process) Sources: GOC:ascb_2009, GOC:dph, GOC:tb Definition: The orderly movement of a chondrocyte from one site to another that contributes to the shaping of growth plate cartilage in an endochondral bone. Relationships: is a type of cell migration [GO:0016477]; is part of growth plate cartilage morphogenesis [GO:0003422]; is part of convergent extension involved in organogenesis [GO:0060029]